{
  "term_label": "malate metabolic process",
  "gene_symbol": "MDH1",
  "gene": "UniProtKB:P40925",
  "term_id": "GO:0006108",
  "gene_name": "Malate dehydrogenase, cytoplasmic"
}